{
  "term_id": "UNKNOWN:0003",
  "gene_symbol": "DUSP14",
  "gene": "UniProtKB:O95147",
  "term_label": "Unknown cellular component",
  "gene_name": "Dual specificity protein phosphatase 14"
}